{
  "gene_symbol": "KCNRG",
  "gene": "UniProtKB:Q8N5I3",
  "gene_name": "Potassium channel regulatory protein",
  "term_id": "UNKNOWN:0002",
  "term_label": "Unknown biological process"
}